negative regulation of appetite by leptin-mediated signaling pathway [GO:0038108] (biological process) Also known as: inhibition of appetite by leptin signaling, negative regulation of appetite by leptin-mediated signalling pathway, reduction of appetite by leptin-mediated signaling, suppression of appetite by leptin-mediated signaling pathway Definition: The series of molecular signals initiated by leptin binding to its receptor on the surface of a cell, which reduces appetite, the desire or physical craving for food. References: PMID:19150989 Sources: GOC:BHF, GOC:vk Relationships: is a type of GO:0032099; is a type of leptin-mediated signaling pathway [GO:0033210]